growth hormone secretion [GO:0030252] (biological process) Sources: GOC:mah Relationships: is a type of peptide hormone secretion [GO:0030072] Also known as: somatotropin secretion Regulation: RO_0002211 by regulation of growth hormone secretion [GO:0060123]; positively regulated by positive regulation of growth hormone secretion [GO:0060124]; negatively regulated by GO:0060125 Definition: The regulated release of growth hormone from secretory granules into the blood.